{
  "gene_symbol": "RTL4",
  "term_id": "UNKNOWN:0002",
  "gene": "UniProtKB:Q6ZR62",
  "term_label": "Unknown biological process",
  "gene_name": "Retrotransposon Gag-like protein 4"
}